{
  "gene_name": "Protein ABHD16B",
  "gene_symbol": "ABHD16B",
  "gene": "UniProtKB:Q9H3Z7",
  "term_id": "GO:0006660",
  "term_label": "phosphatidylserine catabolic process"
}